{
  "term_label": "defense response to bacterium",
  "gene_symbol": "HAMP",
  "term_id": "GO:0042742",
  "gene": "UniProtKB:P81172",
  "gene_name": "Hepcidin"
}